regulation of protein K63-linked ubiquitination [GO:1900044] (biological process) Relationships: is a type of regulation of protein polyubiquitination [GO:1902914]; regulates protein K63-linked ubiquitination [GO:0070534] Also known as: regulation of protein K63-linked polyubiquitination Definition: Any process that modulates the frequency, rate or extent of protein K63-linked ubiquitination. Sources: GOC:TermGenie Subtypes: GO:1900045, GO:1902523